{
  "gene": "UniProtKB:Q5SNT2",
  "gene_symbol": "TMEM201",
  "term_label": "nuclear migration along microtubule",
  "gene_name": "Transmembrane protein 201",
  "term_id": "GO:0030473"
}